uracil transmembrane transport [GO:1903791] (biological process) Relationships: is a type of uracil transport [GO:0015857]; is a type of pyrimidine nucleobase transmembrane transport [GO:1904082] References: PMID:8948441 Sources: GOC:TermGenie, GO_REF:0000069 Definition: The process in which uracil is transported across a membrane. Subtypes: uracil import across plasma membrane [GO:0098721]